{
  "term_label": "regulation of dendrite development",
  "gene_symbol": "SEZ6",
  "gene": "UniProtKB:Q53EL9",
  "term_id": "GO:0050773",
  "gene_name": "Seizure protein 6 homolog"
}